{
  "term_id": "UNKNOWN:0002",
  "term_label": "Unknown biological process",
  "gene_symbol": "CLDN34",
  "gene_name": "Claudin-34",
  "gene": "UniProtKB:H7C241"
}